{
  "gene_symbol": "SLC25A17",
  "gene_name": "Peroxisomal membrane protein PMP34",
  "term_id": "GO:0015228",
  "term_label": "coenzyme A transmembrane transporter activity",
  "gene": "UniProtKB:O43808"
}